hydroxyectoine transmembrane transport [GO:0033308] (biological process) Definition: The directed movement of hydroxyectoine across a membrane by means of some agent such as a transporter or a pore. Sources: GOC:mlg Also known as: hydroxyectoine transport Relationships: is a type of quaternary ammonium group transport [GO:0015697]; is a type of monocarboxylic acid transport [GO:0015718]; is_a organic hydroxy compound transport [GO:0015850]; is a type of carboxylic acid transmembrane transport [GO:1905039]